{
  "gene": "UniProtKB:O95271",
  "gene_name": "Poly [ADP-ribose] polymerase tankyrase-1",
  "term_id": "GO:0070198",
  "gene_symbol": "TNKS",
  "term_label": "protein localization to chromosome, telomeric region"
}